{
  "term_id": "GO:0004040",
  "gene": "UniProtKB:O00519",
  "term_label": "amidase activity",
  "gene_symbol": "FAAH",
  "gene_name": "Fatty-acid amide hydrolase 1"
}